{
  "gene_name": "Spectrin alpha chain, non-erythrocytic 1",
  "gene": "UniProtKB:Q13813",
  "term_id": "GO:0051015",
  "term_label": "actin filament binding",
  "gene_symbol": "SPTAN1"
}